glutamate dehydrogenase complex [GO:1990148] (cellular component) Also known as: L-glutamate dehydrogenase complex, L-glutamate:NADP+ oxidoreductase (deaminating) complex, L-glutamic acid dehydrogenase complex, NAD(P)-glutamate dehydrogenase complex, NAD(P)H-dependent glutamate dehydrogenase complex, dehydrogenase, glutamate (nicotinamide adenine dinucleotide (phosphate)) complex, glutamate dehydrogenase (NADP+) complex, glutamic acid dehydrogenase complex, glutamic dehydrogenase complex Relationships: is a type of oxidoreductase complex [GO:1990204] References: PMID:22393408, PMID:23412807 Sources: GOC:bhm Definition: A homomeric protein complex that possesses glutamate dehydrogenase activity. This complex is evolutionarily conserved except that the number of homoprotomers per complex varies.